{
  "gene_symbol": "RPL30",
  "gene": "UniProtKB:P62888",
  "term_id": "GO:0003735",
  "gene_name": "Large ribosomal subunit protein eL30",
  "term_label": "structural constituent of ribosome"
}